secretory granule organization [GO:0033363] (biological process) Regulation: RO_0002211 by regulation of secretory granule organization [GO:1904409]; negatively regulated by negative regulation of secretory granule organization [GO:1904410]; positively regulated by positive regulation of secretory granule organization [GO:1904411] Relationships: is a type of vesicle organization [GO:0016050]; is part of endomembrane system organization [GO:0010256] Definition: A process that is carried out at the cellular level which results in the assembly, arrangement of constituent parts, or disassembly of a secretory granule. A secretory granule is a small subcellular vesicle, surrounded by a membrane, that is formed from the Golgi apparatus and contains a highly concentrated protein destined for secretion. Subtypes: acrosome assembly [GO:0001675], mast cell secretory granule organization [GO:0033364], T cell secretory granule organization [GO:0033371], platelet dense granule organization [GO:0060155], dense core granule organization [GO:0061109], secretory granule maturation [GO:0061792], platelet alpha granule organization [GO:0070889] Also known as: secretory granule organisation, secretory granule organization and biogenesis Sources: GOC:mah